D-amino acid catabolic process [GO:0019478] (biological process) Relationships: is a type of GO:0046416; is a type of non-proteinogenic amino acid catabolic process [GO:0170044]; is a type of alpha-amino acid catabolic process [GO:1901606] Definition: The chemical reactions and pathways resulting in the breakdown of D-amino acids, the D-enantiomers of amino acids. Sources: GOC:ai, GOC:jsg Also known as: D-amino acid breakdown, D-amino acid catabolism, D-amino acid degradation Subtypes: D-cysteine catabolic process [GO:0019447], GO:0019476, D-serine catabolic process [GO:0036088], D-alanine catabolic process [GO:0055130], D-tyrosine catabolic process [GO:1900829], GO:1900832, GO:1902079